{
  "term_label": "cell redox homeostasis",
  "term_id": "GO:0045454",
  "gene_symbol": "SELENOT",
  "gene": "UniProtKB:P62341",
  "gene_name": "Thioredoxin reductase-like selenoprotein T"
}